{
  "term_id": "GO:0017056",
  "gene_symbol": "POM121B",
  "gene": "UniProtKB:A6NF01",
  "term_label": "structural constituent of nuclear pore",
  "gene_name": "Putative nuclear envelope pore membrane protein POM 121B"
}